{
  "gene_symbol": "DAXX",
  "gene_name": "Death domain-associated protein 6",
  "gene": "UniProtKB:Q9UER7",
  "term_label": "transcription corepressor activity",
  "term_id": "GO:0003714"
}